{
  "gene_symbol": "RIC8A",
  "term_id": "GO:0001965",
  "gene": "UniProtKB:Q9NPQ8",
  "term_label": "G-protein alpha-subunit binding",
  "gene_name": "Synembryn-A"
}